{
  "term_label": "Unknown molecular function",
  "gene": "UniProtKB:Q9H4G0",
  "term_id": "UNKNOWN:0001",
  "gene_symbol": "EPB41L1",
  "gene_name": "Band 4.1-like protein 1"
}